{
  "gene_name": "PAT complex subunit Asterix",
  "gene": "UniProtKB:Q9Y284",
  "term_id": "GO:0045048",
  "gene_symbol": "WDR83OS",
  "term_label": "protein insertion into ER membrane"
}